{
  "gene": "UniProtKB:P18085",
  "gene_symbol": "ARF4",
  "gene_name": "ADP-ribosylation factor 4",
  "term_label": "vesicle-mediated transport",
  "term_id": "GO:0016192"
}